cardiac muscle tissue growth involved in heart morphogenesis [GO:0003245] (biological process) Relationships: is a type of GO:0003241; is a type of cardiac muscle tissue growth [GO:0055017]; is part of GO:0055008 Definition: The developmental growth of cardiac muscle tissue that contributes to the shaping of the heart. Sources: GOC:mtg_heart